{
  "term_id": "GO:0005615",
  "term_label": "extracellular space",
  "gene_symbol": "PON3",
  "gene_name": "Serum paraoxonase_lactonase 3",
  "gene": "UniProtKB:Q15166"
}